{
  "gene": "UniProtKB:Q6ZUL3",
  "term_id": "UNKNOWN:0003",
  "gene_name": "Uncharacterized protein LINC03042",
  "term_label": "Unknown cellular component",
  "gene_symbol": "LINC03042"
}